vesicle tethering to Golgi [GO:0099041] (biological process) References: PMID:27243008 Definition: The initial, indirect interaction between a transport vesicle membrane and the membrane of the Golgi. This interaction is mediated by tethering factors (or complexes), which interact with both membranes. Interaction can occur via direct binding to membrane phospholipids or membrane proteins, or via binding to vesicle coat proteins. This process is distinct from and prior fusion. Relationships: is_a vesicle tethering [GO:0099022]